{
  "gene_symbol": "DCLRE1C",
  "term_label": "telomere maintenance",
  "gene": "UniProtKB:Q96SD1",
  "gene_name": "Protein artemis",
  "term_id": "GO:0000723"
}